{
  "term_id": "UNKNOWN:0002",
  "term_label": "Unknown biological process",
  "gene_symbol": "CSTA",
  "gene": "UniProtKB:P01040",
  "gene_name": "Cystatin-A"
}